{
  "term_label": "synaptic vesicle",
  "gene": "UniProtKB:O95716",
  "term_id": "GO:0008021",
  "gene_name": "Ras-related protein Rab-3D",
  "gene_symbol": "RAB3D"
}